embryo development [GO:0009790] (biological process) Also known as: embryogenesis and morphogenesis, embryogenesis, embryonal development Subtypes: embryo development ending in birth or egg hatching [GO:0009792], GO:0009793, morula development [GO:0014000] Definition: The process whose specific outcome is the progression of an embryo from its formation until the end of its embryonic life stage. The end of the embryonic stage is organism-specific. For example, for mammals, the process would begin with zygote formation and end with birth. For insects, the process would begin at zygote formation and end with larval hatching. For plant zygotic embryos, this would be from zygote formation to the end of seed dormancy. For plant vegetative embryos, this would be from the initial determination of the cell or group of cells to form an embryo until the point when the embryo becomes independent of the parent plant. Regulation: positively regulated by positive regulation of embryonic development [GO:0040019]; negatively regulated by negative regulation of embryonic development [GO:0045992]; regulated by GO:0045995 Relationships: is a type of GO:0007275 Sources: GOC:go_curators, GOC:isa_complete, GOC:mtg_sensu